{
  "gene": "UniProtKB:Q96JP2",
  "gene_symbol": "MYO15B",
  "gene_name": "Unconventional myosin-XVB",
  "term_id": "UNKNOWN:0001",
  "term_label": "Unknown molecular function"
}